{
  "gene": "UniProtKB:Q5VTD9",
  "term_id": "GO:0005634",
  "gene_symbol": "GFI1B",
  "gene_name": "Zinc finger protein Gfi-1b",
  "term_label": "nucleus"
}